{
  "term_label": "Unknown molecular function",
  "gene_symbol": "SPATA21",
  "term_id": "UNKNOWN:0001",
  "gene_name": "Spermatogenesis-associated protein 21",
  "gene": "UniProtKB:Q7Z572"
}